{
  "gene_name": "Mdm2-binding protein",
  "gene_symbol": "MTBP",
  "term_label": "Unknown molecular function",
  "term_id": "UNKNOWN:0001",
  "gene": "UniProtKB:Q96DY7"
}